{
  "gene_symbol": "CLK4",
  "term_label": "protein tyrosine kinase activity",
  "term_id": "GO:0004713",
  "gene_name": "Dual specificity protein kinase CLK4",
  "gene": "UniProtKB:Q9HAZ1"
}